{
  "gene_symbol": "KCNE5",
  "term_id": "GO:0060307",
  "gene_name": "Potassium voltage-gated channel subfamily E regulatory beta subunit 5",
  "gene": "UniProtKB:Q9UJ90",
  "term_label": "regulation of ventricular cardiac muscle cell membrane repolarization"
}